{
  "term_label": "monoacylglycerol lipase activity",
  "gene": "UniProtKB:Q8WU67",
  "gene_symbol": "ABHD3",
  "gene_name": "Phospholipase ABHD3",
  "term_id": "GO:0047372"
}